{
  "gene_symbol": "OLFML1",
  "term_id": "GO:0007165",
  "gene_name": "Olfactomedin-like protein 1",
  "term_label": "signal transduction",
  "gene": "UniProtKB:Q6UWY5"
}